{
  "gene": "UniProtKB:Q9GZT8",
  "gene_symbol": "NIF3L1",
  "term_id": "GO:0005739",
  "gene_name": "NIF3-like protein 1",
  "term_label": "mitochondrion"
}